{
  "gene": "UniProtKB:P20933",
  "gene_symbol": "AGA",
  "term_id": "GO:0005737",
  "gene_name": "N(4)-(beta-N-acetylglucosaminyl)-L-asparaginase",
  "term_label": "cytoplasm"
}